{
  "gene": "UniProtKB:Q9HB66",
  "term_label": "Unknown cellular component",
  "gene_symbol": "MKKS",
  "term_id": "UNKNOWN:0003",
  "gene_name": "Alternative protein MKKS"
}